{
  "term_label": "Unknown cellular component",
  "gene_name": "Putative G antigen family E member 3",
  "gene": "UniProtKB:Q5JRK9",
  "gene_symbol": "PAGE2B",
  "term_id": "UNKNOWN:0003"
}